chalcone isomerase activity [GO:0045430] (molecular function) Also known as: chalcone-flavanone isomerase activity, chalcone--flavonone isomerase activity, flavanone lyase (decyclizing) Relationships: is a type of intramolecular lyase activity [GO:0016872] Sources: EC:5.5.1.6 Definition: Catalysis of the reaction: a chalcone = a flavanone.